{
  "gene": "UniProtKB:O14529",
  "gene_symbol": "CUX2",
  "term_id": "GO:0006357",
  "term_label": "regulation of transcription by RNA polymerase II",
  "gene_name": "Homeobox protein cut-like 2"
}